succinate-CoA ligase activity [GO:0004774] (molecular function) Definition: Catalysis of the reaction: succinate + CoA + nucleotide triphosphate = nucleotide diphosphate + phosphate + succinyl-CoA. Subtypes: succinate-CoA ligase (ADP-forming) activity [GO:0004775], succinate-CoA ligase (GDP-forming) activity [GO:0004776] Sources: GOC:ai Relationships: is a type of acid-thiol ligase activity [GO:0016878]